{
  "gene": "UniProtKB:Q9BZD4",
  "gene_name": "Kinetochore protein Nuf2",
  "gene_symbol": "NUF2",
  "term_label": "Ndc80 complex",
  "term_id": "GO:0031262"
}